osmoregulated periplasmic glucan biosynthetic process [GO:1900727] (BP) Definition: The chemical reactions and pathways resulting in the formation of osmoregulated periplasmic glucan. Relationships: is a type of glucan biosynthetic process [GO:0009250] Also known as: osmoregulated periplasmic glucan anabolism, osmoregulated periplasmic glucan biosynthesis, osmoregulated periplasmic glucan formation, osmoregulated periplasmic glucan synthesis Sources: GOC:TermGenie, GOC:yaf